{
  "gene_symbol": "DNASE2B",
  "term_id": "GO:0006309",
  "term_label": "apoptotic DNA fragmentation",
  "gene": "UniProtKB:Q8WZ79",
  "gene_name": "Deoxyribonuclease-2-beta"
}